{
  "gene": "UniProtKB:Q86UG4",
  "term_id": "GO:0043252",
  "gene_name": "Solute carrier organic anion transporter family member 6A1",
  "gene_symbol": "SLCO6A1",
  "term_label": "sodium-independent organic anion transport"
}